peptidyl-lysine propionylation [GO:0061921] (biological process) Definition: The propionylation of peptidyl-lysine. Relationships: is a type of protein acylation [GO:0043543] References: PMID:17267393